{
  "term_label": "Unknown cellular component",
  "term_id": "UNKNOWN:0003",
  "gene_name": "Testis-specific serine_threonine-protein kinase 6",
  "gene": "UniProtKB:Q9BXA6",
  "gene_symbol": "TSSK6"
}